{
  "gene_name": "Histone-lysine N-methyltransferase MECOM",
  "gene": "UniProtKB:Q03112",
  "gene_symbol": "MECOM",
  "term_label": "regulation of transcription by RNA polymerase II",
  "term_id": "GO:0006357"
}